{
  "term_id": "GO:0006886",
  "gene_symbol": "RAB23",
  "gene_name": "Ras-related protein Rab-23",
  "gene": "UniProtKB:Q9ULC3",
  "term_label": "intracellular protein transport"
}